streptomycin-6-phosphatase activity [GO:0050301] (molecular function) Definition: Catalysis of the reaction: H2O + streptomycin 6-phosphate = phosphate + streptomycin. Sources: EC:3.1.3.39, RHEA:10688 Relationships: is a type of phosphatase activity [GO:0016791] Also known as: streptomycin 6-phosphate phosphatase activity, streptomycin 6-phosphate phosphohydrolase activity, streptomycin-6-P phosphohydrolase activity, streptomycin-6-phosphate phosphohydrolase activity